RNA NAD-cap (NMN-forming) hydrolase activity [GO:0110153] (molecular function) Definition: Catalysis of the reaction: a 5'-end NAD+-phospho-ribonucleoside in mRNA + H2O = a 5'-end phospho-adenosine-phospho-ribonucleoside in mRNA + beta-nicotinamide D-ribonucleotide + 2 H+. Relationships: is a type of pyrophosphatase activity [GO:0016462]; is a type of catalytic activity, acting on RNA [GO:0140098] References: PMID:25533955, PMID:31101919 Sources: GOC:sp, RHEA:60876 Note: This reaction specifically removes the nicotinamide adenine dinucleotide (NAD) cap from a subset of mRNAs by hydrolyzing the diphosphate linkage to produce nicotinamide mononucleotide (NMN) and 5' monophosphate mRNA.